glucosaminate ammonia-lyase activity [GO:0047930] (molecular function) Definition: Catalysis of the reaction: D-glucosaminate = 2-dehydro-3-deoxy-D-gluconate + NH3. Relationships: is a type of ammonia-lyase activity [GO:0016841] Sources: EC:4.3.1.9 Note: Note that this function was EC:4.3.1.21. Also known as: aminodeoxygluconate ammonia-lyase activity, aminodeoxygluconate dehydratase activity, 2-amino-2-deoxy-D-gluconate ammonia-lyase activity, 2-amino-2-deoxy-D-gluconate hydro-lyase (deaminating) activity, D-glucosaminate ammonia-lyase (isomerizing; 2-dehydro-3-deoxy-D-gluconate-forming), D-glucosaminate ammonia-lyase activity, D-glucosaminate dehydratase activity, D-glucosaminic acid dehydrase activity, acetylenemonocarboxylic acid hydrase activity, glucosaminic dehydrase activity